{
  "gene_name": "Nuclear receptor subfamily 0 group B member 1",
  "gene_symbol": "NR0B1",
  "term_label": "transcription corepressor activity",
  "gene": "UniProtKB:P51843",
  "term_id": "GO:0003714"
}